{
  "gene_name": "Protein eva-1 homolog C",
  "term_id": "UNKNOWN:0002",
  "gene": "UniProtKB:P58658",
  "term_label": "Unknown biological process",
  "gene_symbol": "EVA1C"
}